{
  "term_label": "regulation of transcription by RNA polymerase II",
  "gene": "UniProtKB:P23760",
  "gene_symbol": "PAX3",
  "term_id": "GO:0006357",
  "gene_name": "Paired box protein Pax-3"
}